{
  "gene_name": "Rho-related BTB domain-containing protein 2",
  "term_id": "GO:0019901",
  "term_label": "protein kinase binding",
  "gene_symbol": "RHOBTB2",
  "gene": "UniProtKB:Q9BYZ6"
}